{
  "gene_symbol": "PISD",
  "term_label": "phosphatidylethanolamine biosynthetic process",
  "gene_name": "Phosphatidylserine decarboxylase proenzyme, mitochondrial",
  "gene": "UniProtKB:Q9UG56",
  "term_id": "GO:0006646"
}